negative regulation of eosinophil chemotaxis [GO:2000423] (BP) Definition: Any process that stops, prevents or reduces the frequency, rate or extent of eosinophil chemotaxis. Sources: GOC:obol Relationships: is_a negative regulation of granulocyte chemotaxis [GO:0071623]; is a type of GO:2000417; is a type of regulation of eosinophil chemotaxis [GO:2000422]; negatively regulates eosinophil chemotaxis [GO:0048245]